stress granule disassembly [GO:0035617] (biological process) Also known as: SG disassembly References: PMID:19825938 Sources: GOC:BHF Relationships: is a type of protein-RNA complex disassembly [GO:0032988]; is a type of organelle disassembly [GO:1903008] Definition: The disaggregation of a stress granule into its constituent protein and RNA parts.